myoblast fate commitment involved in skeletal muscle regeneration [GO:0014836] (biological process) Definition: The process in which the developmental fate of a satellite cell becomes restricted such that it will develop into a myoblast. This occurs as part of skeletal muscle regeneration. A myoblast is a mononucleate cell type that, by fusion with other myoblasts, gives rise to the myotubes that eventually develop into skeletal muscle fibers. References: PMID:16607119 Sources: CL:0000056, GOC:ef, GOC:mtg_muscle Relationships: is a type of myoblast fate commitment [GO:0048625]; is part of myoblast differentiation involved in skeletal muscle regeneration [GO:0014835]